positive regulation of mammary placode formation by mesenchymal-epithelial signaling [GO:0060617] (biological process) Relationships: is a type of GO:0022603; is a type of positive regulation of developmental process [GO:0051094]; is a type of GO:0051240; is a type of mesenchymal-epithelial cell signaling [GO:0060638]; is a type of regulation of multicellular organismal development [GO:2000026]; positively regulates mammary placode formation [GO:0060596] Also known as: positive regulation of mammary placode formation by mesenchymal-epithelial signalling Definition: Any process that initiates the formation of a mammary placode through a mechanism that mediates the transfer of information from a mesenchymal cell to an epithelial cell resulting in the epithelial cell adopting the identity of a cell of the mammary placode. References: PMID:12558599 Sources: GOC:dph